{
  "term_id": "GO:0005886",
  "gene": "UniProtKB:P48995",
  "gene_symbol": "TRPC1",
  "gene_name": "Short transient receptor potential channel 1",
  "term_label": "plasma membrane"
}